RNA polymerase III transcription regulator complex [GO:0090576] (cellular component) Sources: GOC:tb Relationships: is a type of transcription regulator complex [GO:0005667] Subtypes: transcription factor TFIIIB complex [GO:0000126], transcription factor TFIIIC complex [GO:0000127], GO:0034734, GO:0034735, TFIIIC-TOP1-SUB1 complex [GO:0034740], transcription factor TFIIIE complex [GO:0070264] Definition: A transcription factor complex that acts at a regulatory region of a gene transcribed by RNA polymerase III. Also known as: RNA polymerase III transcription factor complex